{
  "gene": "UniProtKB:Q9BS86",
  "term_label": "acrosomal vesicle",
  "term_id": "GO:0001669",
  "gene_symbol": "ZPBP",
  "gene_name": "Zona pellucida-binding protein 1"
}